{
  "term_id": "GO:0008202",
  "gene_name": "Cytochrome P450 3A7",
  "gene_symbol": "CYP3A7",
  "term_label": "steroid metabolic process",
  "gene": "UniProtKB:P24462"
}